{
  "gene_symbol": "TMEM64",
  "gene": "UniProtKB:Q6YI46",
  "term_id": "GO:0045672",
  "term_label": "positive regulation of osteoclast differentiation",
  "gene_name": "Transmembrane protein 64"
}